{
  "gene_symbol": "CGB3",
  "term_id": "GO:0007186",
  "term_label": "G protein-coupled receptor signaling pathway",
  "gene_name": "Choriogonadotropin subunit beta 3",
  "gene": "UniProtKB:P0DN86"
}